regulation of cell proliferation involved in kidney morphogenesis [GO:0061006] (biological process) Definition: Any process that modulates the frequency, rate or extent of cell proliferation that contributes to the shaping of the kidney. Relationships: is a type of GO:0042127; is part of kidney morphogenesis [GO:0060993] Sources: GOC:dph, GOC:mtg_kidney_jan10